positive regulation of peptidyl-lysine acetylation [GO:2000758] (biological process) Definition: Any process that activates or increases the frequency, rate or extent of peptidyl-lysine acetylation. Subtypes: positive regulation of N-terminal peptidyl-lysine acetylation [GO:2000761] Relationships: is a type of GO:1901985; is a type of regulation of peptidyl-lysine acetylation [GO:2000756]; positively regulates peptidyl-lysine acetylation [GO:0018394] Sources: GOC:obol